somatostatin binding [GO:0120023] (molecular function) Definition: Binding to somatostatin, a polypeptide hormone involved in regulating pancreatic alpha and pancreatic beta cells and controlling growth hormone secretion as well as many other functions. Somatostatin is produced by several cell types including pancreatic delta cells. There are several different mature forms of somatostatin. References: PMID:20472043 Sources: GOC:cvs Relationships: is a type of peptide hormone binding [GO:0017046]